mesonephric tubule development [GO:0072164] (biological process) Relationships: is a type of tube development [GO:0035295]; is a type of mesonephric epithelium development [GO:0072163] Sources: GOC:mtg_kidney_jan10 Subtypes: ureteric bud development [GO:0001657], mesonephric nephron tubule development [GO:0061242], anterior mesonephric tubule development [GO:0072165], posterior mesonephric tubule development [GO:0072166], mesonephric duct development [GO:0072177] Definition: The progression of a mesonephric tubule over time, from its initial formation to the mature structure. A mesonephric tubule is an epithelial tube that is part of the mesonephros.